{
  "gene": "UniProtKB:O00194",
  "term_id": "GO:0045921",
  "gene_name": "Ras-related protein Rab-27B",
  "term_label": "positive regulation of exocytosis",
  "gene_symbol": "RAB27B"
}